{
  "gene": "UniProtKB:P20366",
  "term_label": "tachykinin receptor signaling pathway",
  "gene_symbol": "TAC1",
  "gene_name": "Protachykinin-1",
  "term_id": "GO:0007217"
}